{
  "term_id": "GO:0005829",
  "gene_name": "Hexokinase-1",
  "gene": "UniProtKB:P19367",
  "gene_symbol": "HK1",
  "term_label": "cytosol"
}